specification of plant organ position [GO:0090706] (biological process) Definition: The regionalization process in which information that determines the correct position at which plant organ primordia are formed is generated and perceived resulting in correct positioning of the new plant organ. References: PMID:9611175 Sources: GOC:tb Relationships: is a type of regionalization [GO:0003002]; BFO_0000050 plant organ morphogenesis [GO:1905392]